{
  "gene_name": "NADPH oxidase 5",
  "term_label": "superoxide-generating NAD(P)H oxidase activity",
  "gene_symbol": "NOX5",
  "term_id": "GO:0016175",
  "gene": "UniProtKB:Q96PH1"
}